{
  "term_label": "endoplasmic reticulum",
  "gene_name": "Membrane primary amine oxidase",
  "term_id": "GO:0005783",
  "gene": "UniProtKB:Q16853",
  "gene_symbol": "AOC3"
}